{
  "gene_name": "Olfactory receptor 5H8",
  "gene_symbol": "OR5H8",
  "gene": "UniProtKB:P0DN80",
  "term_label": "Unknown biological process",
  "term_id": "UNKNOWN:0002"
}